{
  "term_id": "GO:0015501",
  "gene_symbol": "SLC1A3",
  "gene": "UniProtKB:P43003",
  "gene_name": "Excitatory amino acid transporter 1",
  "term_label": "glutamate:sodium symporter activity"
}